{
  "term_label": "T cell costimulation",
  "term_id": "GO:0031295",
  "gene_name": "T-cell-specific surface glycoprotein CD28",
  "gene_symbol": "CD28",
  "gene": "UniProtKB:P10747"
}